{
  "gene_name": "DnaJ homolog subfamily C member 24",
  "term_id": "UNKNOWN:0002",
  "term_label": "Unknown biological process",
  "gene": "UniProtKB:Q6P3W2",
  "gene_symbol": "DNAJC24"
}